{
  "gene": "UniProtKB:P09496",
  "gene_name": "Clathrin light chain A",
  "gene_symbol": "CLTA",
  "term_label": "clathrin heavy chain binding",
  "term_id": "GO:0032050"
}